Y chromosome [GO:0000806] (cellular component) Relationships: is a type of sex chromosome [GO:0000803] Definition: The sex chromosome present in males of species in which the male is the heterogametic sex; generally, the sex chromosome that pairs with the X chromosome in the heterogametic sex. The Y chromosome is absent from the cells of females and present in one copy in the somatic cells of males. References: PMID:20622855 Sources: GOC:mah, GOC:mr, ISBN:0582227089, Wikipedia:XY_sex-determination_system